endoplasmic reticulum inheritance [GO:0048309] (biological process) Definition: The partitioning of endoplasmic reticulum between daughter cells at cell division. Sources: GOC:jid Relationships: is a type of GO:0007029; is a type of GO:0048308 Also known as: ER inheritance